Sin3-type complex [GO:0070822] (cellular component) Definition: Any of a number of evolutionarily conserved histone deacetylase complexes (HDACs) containing a core consisting of a paired amphipathic helix motif protein (e.g. Sin3p in S. cerevisiae, Pst1 in S. pombe or Sin3A in mammals) at least one class I histone deacetylase (e.g. Rpd3p in S. cerevisiae, Clr6 in S. pombe, or HDAC1 and HDAC2 in mammals), and at least one WD40 repeat protein (e.g. Ume1p in S. cerevisiae, Prw1 in S. pombe, or RbAp46 and RbAp48 in mammals). These complexes also contain a variable number of other proteins that direct histone binding, DNA binding, or add other functionality to the complex. References: PMID:15565322, PMID:18292778 Relationships: is a type of GO:0000118; is part of nuclear chromosome [GO:0000228]; is part of GO:0000785 Subtypes: Rpd3S complex [GO:0032221], Rpd3L complex [GO:0033698]